{
  "term_label": "positive regulation of cell migration",
  "term_id": "GO:0030335",
  "gene_name": "Semaphorin-7A",
  "gene": "UniProtKB:O75326",
  "gene_symbol": "SEMA7A"
}